{
  "term_id": "GO:0002161",
  "term_label": "aminoacyl-tRNA deacylase activity",
  "gene": "UniProtKB:Q5JTZ9",
  "gene_name": "Alanine--tRNA ligase, mitochondrial",
  "gene_symbol": "AARS2"
}